negative regulation of defecation [GO:2000293] (BP) Definition: Any process that stops, prevents or reduces the frequency, rate or extent of defecation. Subtypes: negative regulation of defecation rhythm [GO:2000747] Sources: GOC:obol Relationships: is a type of negative regulation of secretion [GO:0051048]; is a type of GO:0060457; is a type of regulation of defecation [GO:2000292]; negatively regulates defecation [GO:0030421]